{
  "term_label": "regulation of T cell activation",
  "gene_symbol": "SIT1",
  "gene_name": "Signaling threshold-regulating transmembrane adapter 1",
  "term_id": "GO:0050863",
  "gene": "UniProtKB:Q9Y3P8"
}